{
  "gene_symbol": "TRIM36",
  "term_id": "GO:0001669",
  "gene_name": "E3 ubiquitin-protein ligase TRIM36",
  "term_label": "acrosomal vesicle",
  "gene": "UniProtKB:Q9NQ86"
}